regulation of natural killer cell activation [GO:0032814] (biological process) Definition: Any process that modulates the frequency, rate or extent of natural killer cell activation. Also known as: regulation of NK cell activation Relationships: is a type of regulation of lymphocyte activation [GO:0051249]; regulates natural killer cell activation [GO:0030101] Subtypes: negative regulation of natural killer cell activation [GO:0032815], positive regulation of natural killer cell activation [GO:0032816], regulation of natural killer cell proliferation [GO:0032817], GO:0032823 Sources: GOC:mah